{
  "gene": "UniProtKB:P10914",
  "gene_name": "Interferon regulatory factor 1",
  "gene_symbol": "IRF1",
  "term_label": "regulation of transcription by RNA polymerase II",
  "term_id": "GO:0006357"
}